{
  "gene": "UniProtKB:Q6IC83",
  "gene_symbol": "C22orf42",
  "gene_name": "Uncharacterized protein C22orf42",
  "term_label": "Unknown biological process",
  "term_id": "UNKNOWN:0002"
}